positive regulation of assembly of large subunit precursor of preribosome [GO:1902628] (biological process) Definition: Any process that activates or increases the frequency, rate or extent of assembly of a large subunit precursor of preribosome. References: PMID:22735702 Sources: GOC:TermGenie, GOC:di, GO_REF:0000058 Also known as: positive regulation of preribosome, large subunit precursor formation, up regulation of assembly of large subunit precursor of preribosome, up regulation of preribosome, large subunit precursor formation, up-regulation of assembly of large subunit precursor of preribosome, up-regulation of preribosome, large subunit precursor formation, upregulation of assembly of large subunit precursor of preribosome, upregulation of preribosome, large subunit precursor formation, activation of 66S preribosome assembly, activation of 66S preribosome formation, activation of assembly of large subunit precursor of preribosome, activation of preribosome, large subunit precursor formation, positive regulation of 66S preribosome assembly, positive regulation of 66S preribosome formation, up regulation of 66S preribosome assembly, up regulation of 66S preribosome formation, up-regulation of 66S preribosome assembly, up-regulation of 66S preribosome formation, upregulation of 66S preribosome assembly, upregulation of 66S preribosome formation Relationships: is a type of positive regulation of protein-containing complex assembly [GO:0031334]; is a type of regulation of assembly of large subunit precursor of preribosome [GO:1902627]; positively regulates assembly of large subunit precursor of preribosome [GO:1902626]